mRNA 5'-triphosphate monophosphatase activity [GO:0140818] (molecular function) Relationships: is a type of pyrophosphatase activity [GO:0016462]; is a type of catalytic activity, acting on RNA [GO:0140098] Definition: A 5'-end triphospho-[mRNA] + H2O = a 5'-end diphospho-[mRNA] + H+ + phosphate. Regulation: RO_0002213 by GO:0170008 Also known as: mRNA 5'-phosphatase activity References: PMID:9473487